{
  "term_label": "nucleus",
  "gene_symbol": "ZNF813",
  "gene": "UniProtKB:Q6ZN06",
  "term_id": "GO:0005634",
  "gene_name": "Zinc finger protein 813"
}